{
  "gene": "UniProtKB:Q3LHN2",
  "term_id": "UNKNOWN:0002",
  "gene_name": "Keratin-associated protein 19-2",
  "gene_symbol": "KRTAP19-2",
  "term_label": "Unknown biological process"
}